oxylipin biosynthetic process [GO:0031408] (biological process) Definition: The chemical reactions and pathways resulting in the formation of any oxylipin, any of a group of biologically active compounds formed by oxidative metabolism of polyunsaturated fatty acids. References: PMID:11960741 Sources: GOC:mah Also known as: oxylipin anabolism, oxylipin biosynthesis, oxylipin formation, oxylipin synthesis Relationships: is a type of oxylipin metabolic process [GO:0031407]; is a type of carboxylic acid biosynthetic process [GO:0046394]